{
  "gene_symbol": "OR4A15",
  "gene": "UniProtKB:Q8NGL6",
  "gene_name": "Olfactory receptor 4A15",
  "term_id": "GO:0004984",
  "term_label": "olfactory receptor activity"
}